positive regulation of L-proline catabolic process to L-glutamate [GO:2001158] (biological process) Also known as: positive regulation of proline catabolic process to glutamate, positive regulation of proline breakdown to glutamate, positive regulation of proline degradation to glutamate, positive regulation of proline oxidation Relationships: is a type of positive regulation of catabolic process [GO:0009896]; is a type of positive regulation of amino acid metabolic process [GO:0045764]; is a type of positive regulation of small molecule metabolic process [GO:0062013]; is a type of regulation of L-proline catabolic process to L-glutamate [GO:2001156]; positively regulates GO:0010133 Definition: Any process that activates or increases the frequency, rate or extent of L-proline catabolic process to glutamate. Sources: GOC:obol